{
  "gene_name": "Gamma-soluble NSF attachment protein",
  "gene_symbol": "NAPG",
  "term_id": "GO:0005483",
  "gene": "UniProtKB:Q99747",
  "term_label": "soluble NSF attachment protein activity"
}